{
  "gene": "UniProtKB:Q9Y3D3",
  "gene_symbol": "MRPS16",
  "gene_name": "Small ribosomal subunit protein bS16m",
  "term_label": "structural constituent of ribosome",
  "term_id": "GO:0003735"
}